{
  "term_label": "RNA polymerase II general transcription initiation factor activity",
  "gene": "UniProtKB:Q6P1X5",
  "gene_name": "Transcription initiation factor TFIID subunit 2",
  "gene_symbol": "TAF2",
  "term_id": "GO:0016251"
}